{
  "gene": "UniProtKB:Q8IUZ0",
  "gene_name": "Leucine-rich repeat-containing protein 49",
  "gene_symbol": "LRRC49",
  "term_label": "Unknown molecular function",
  "term_id": "UNKNOWN:0001"
}